{
  "term_label": "GTP binding",
  "gene_name": "Rho-related GTP-binding protein RhoF",
  "gene": "UniProtKB:Q9HBH0",
  "term_id": "GO:0005525",
  "gene_symbol": "RHOF"
}